{
  "gene_name": "Kelch domain-containing protein 7B",
  "gene_symbol": "KLHDC7B",
  "gene": "UniProtKB:Q96G42",
  "term_label": "Unknown molecular function",
  "term_id": "UNKNOWN:0001"
}